cell-cell signaling via exosome [GO:0099156] (biological process) Subtypes: trans-synaptic signaling via exosome [GO:0099157] Relationships: is_a cell-cell signaling [GO:0007267] References: PMID:19837038 Sources: GOC:dos Also known as: exosome mediated Definition: Cell-cell signaling in which the ligand is carried between cells by an exosome.